8-oxo-GDP phosphatase activity [GO:0044716] (MF) Definition: Catalysis of the reaction 8-oxo-GDP + H2O = 8-oxo-GMP + phosphate. References: PMID:22556419 Sources: GOC:pde, RHEA:62356 Relationships: is a type of nucleoside diphosphate phosphatase activity [GO:0017110]